IMP salvage [GO:0032264] (biological process) Definition: Any process which produces inosine monophosphate from derivatives of it, without de novo synthesis. Sources: GOC:mah Relationships: is a type of IMP biosynthetic process [GO:0006188]; is a type of purine ribonucleotide salvage [GO:0106380]